{
  "gene_name": "Zinc finger protein 469",
  "term_id": "UNKNOWN:0002",
  "term_label": "Unknown biological process",
  "gene": "UniProtKB:Q96JG9",
  "gene_symbol": "ZNF469"
}